{
  "gene_name": "Protocadherin-15",
  "term_label": "plasma membrane",
  "term_id": "GO:0005886",
  "gene_symbol": "PCDH15",
  "gene": "UniProtKB:Q96QU1"
}